{
  "gene_name": "TPR and ankyrin repeat-containing protein 1",
  "gene_symbol": "TRANK1",
  "term_label": "Unknown molecular function",
  "term_id": "UNKNOWN:0001",
  "gene": "UniProtKB:O15050"
}